{
  "gene": "UniProtKB:Q6ZS52",
  "gene_name": "Putative uncharacterized protein FLJ45825",
  "term_id": "UNKNOWN:0001",
  "gene_symbol": "Q6ZS52",
  "term_label": "Unknown molecular function"
}